{
  "term_id": "GO:0000492",
  "gene": "UniProtKB:Q9Y230",
  "gene_symbol": "RUVBL2",
  "term_label": "box C/D snoRNP assembly",
  "gene_name": "RuvB-like 2"
}